{
  "term_label": "Ras protein signal transduction",
  "term_id": "GO:0007265",
  "gene": "UniProtKB:Q07889",
  "gene_symbol": "SOS1",
  "gene_name": "Son of sevenless homolog 1"
}